extracellular structure organization [GO:0043062] (biological process) Relationships: is a type of cellular component organization [GO:0016043] Also known as: extracellular structure organisation, extracellular structure organization and biogenesis Sources: GOC:ai, GOC:dph, GOC:jl, GOC:mah Subtypes: extracellular matrix organization [GO:0030198], intercellular bridge organization [GO:0043063] Definition: A process that is carried out at the cellular level which results in the assembly, arrangement of constituent parts, or disassembly of structures in the space external to the outermost structure of a cell. For cells without external protective or external encapsulating structures this refers to space outside of the plasma membrane, and also covers the host cell environment outside an intracellular parasite.